GDP-D-rhamnose biosynthetic process [GO:0019306] (biological process) Also known as: GDP-D-rhamnose anabolism, GDP-D-rhamnose biosynthesis, GDP-D-rhamnose formation, GDP-D-rhamnose synthesis Sources: GOC:ai Definition: The chemical reactions and pathways resulting in the formation of GDP-D-rhamnose, a substance composed of rhamnose in glycosidic linkage with guanosine diphosphate. Relationships: is a type of nucleotide-sugar biosynthetic process [GO:0009226]